{
  "gene": "UniProtKB:Q9Y240",
  "gene_name": "C-type lectin domain family 11 member A",
  "gene_symbol": "CLEC11A",
  "term_id": "GO:0001503",
  "term_label": "ossification"
}